ferroxidase activity [GO:0004322] (molecular function) Definition: Catalysis of the reaction: 4 Fe2+ + 4 H+ + O2 = 4 Fe3+ + 2 H2O. Sources: RHEA:11148 Also known as: HEPH, caeruloplasmin, ceruloplasmin, hephaestin, multicopper ferroxidase iron transport mediator activity, Fe(II):oxygen oxidoreductase activity, ferro:O2 oxidoreductase activity, ferroxidase I, ferroxidase, iron II:oxygen oxidoreductase activity, iron(II): oxygen oxidoreductase activity Relationships: is a type of oxidoreductase activity, acting on metal ions, oxygen as acceptor [GO:0016724]